{
  "term_label": "guanyl-nucleotide exchange factor activity",
  "gene_symbol": "CYTH3",
  "gene": "UniProtKB:O43739",
  "gene_name": "Cytohesin-3",
  "term_id": "GO:0005085"
}